{
  "term_label": "Unknown biological process",
  "gene_symbol": "NDUFB2",
  "gene_name": "NADH dehydrogenase [ubiquinone] 1 beta subcomplex subunit 2, mitochondrial",
  "gene": "UniProtKB:O95178",
  "term_id": "UNKNOWN:0002"
}